{
  "term_label": "animal organ development",
  "term_id": "GO:0048513",
  "gene": "UniProtKB:O43763",
  "gene_symbol": "TLX2",
  "gene_name": "T-cell leukemia homeobox protein 2"
}